amide catabolic process [GO:0043605] (biological process) Sources: GOC:curators Definition: The chemical reactions and pathways resulting in the breakdown of an amide, any derivative of an oxoacid in which an acidic hydroxy group has been replaced by an amino or substituted amino group. Relationships: is a type of catabolic process [GO:0009056]; is a type of amide metabolic process [GO:0043603] Also known as: cellular amide catabolic process Regulation: RO_0002211 by regulation of amide catabolic process [GO:0034251]; negatively regulated by GO:0034252; positively regulated by positive regulation of amide catabolic process [GO:0034253] Subtypes: GO:0000256, L-asparagine biosynthetic process from oxaloacetate [GO:0019266], GO:0019442, GO:0019457, L-lysine catabolic process to acetyl-CoA [GO:0019474], L-histidine catabolic process to glutamate and formamide [GO:0019556], atrazine catabolic process to urea [GO:0019623], biotin catabolic process [GO:0042367], urea catabolic process [GO:0043419], GO:0070690